cellular response to Gentian violet [GO:0072729] (biological process) Definition: Any process that results in a change in state or activity of a cell (in terms of movement, secretion, enzyme production, gene expression, etc.) as a result of a Gentian violet stimulus. Relationships: is a type of cellular response to chemical stimulus [GO:0070887]; is a type of response to Gentian violet [GO:0072728] Also known as: cellular response to crystal violet, cellular response to {4-[Bis-(4-dimethylamino-phenyl)-methylene]-cyclohexa-2,5-dienylidene}-dimethyl-ammonium chloride Sources: GOC:mah